ciliary neurotrophic factor-mediated signaling pathway [GO:0070120] (biological process) Also known as: CNTF-mediated signaling pathway, ciliary neurotrophic factor-mediated signalling pathway Relationships: is a type of cytokine-mediated signaling pathway [GO:0019221] Sources: GOC:BHF, GOC:mah Definition: The series of molecular signals initiated by the binding of a ciliary neurotrophic factor (CNTF) to its receptor on the surface of a target cell, and ending with the regulation of a downstream cellular process, e.g. transcription.